negative regulation of vascular wound healing [GO:0061044] (BP) Definition: Any process that decreases the rate, frequency, or extent of blood vessel formation when new vessels emerge from the proliferation of pre-existing blood vessels and contribute to the series of events that restore integrity to damaged vasculature. Relationships: is_a GO:0016525; is a type of regulation of vascular wound healing [GO:0061043]; is a type of negative regulation of wound healing [GO:0061045]; negatively regulates vascular wound healing [GO:0061042] Sources: GOC:BHF, GOC:dph